{
  "term_label": "vacuolar acidification",
  "gene_name": "V-type proton ATPase 116 kDa subunit a 2",
  "gene": "UniProtKB:Q9Y487",
  "gene_symbol": "ATP6V0A2",
  "term_id": "GO:0007035"
}